negative regulation of oxidative phosphorylation [GO:0090324] (biological process) Sources: GOC:BHF Relationships: is a type of GO:0002082; is a type of GO:1901856; negatively regulates GO:0006119 Subtypes: negative regulation of mitochondrial ATP synthesis coupled electron transport [GO:1905447] Definition: Any process that decreases the frequency, rate or extent of the chemical reactions and pathways resulting in the phosphorylation of ADP to ATP that accompanies the oxidation of a metabolite through the operation of the respiratory chain. Oxidation of compounds establishes a proton gradient across the membrane, providing the energy for ATP synthesis.